{
  "gene_symbol": "H2BC26",
  "gene_name": "Histone H2B type 3-B",
  "term_id": "GO:0002227",
  "term_label": "innate immune response in mucosa",
  "gene": "UniProtKB:Q8N257"
}